inositol phosphate phosphatase activity [GO:0052745] (MF) Sources: GOC:ai Definition: Catalysis of the reaction: inositol phosphate(n) + H2O = inositol phosphate(n-1) + phosphate. This reaction is the removal of a phosphate group from an inositol phosphate. Relationships: is a type of phosphatase activity [GO:0016791] Subtypes: inositol hexakisphosphate phosphatase activity [GO:0004446], inositol bisphosphate phosphatase activity [GO:0016312], inositol trisphosphate phosphatase activity [GO:0046030], inositol tetrakisphosphate phosphatase activity [GO:0052743], inositol pentakisphosphate phosphatase activity [GO:0052827], inositol monophosphate phosphatase activity [GO:0052834]